serotonin-gated cation-selective signaling pathway [GO:0140227] (biological process) Definition: The series of molecular signals initiated by serotonin binding to a seratonin receptor on the surface of the target cell, followed by the movement of ions through a channel in the receptor complex. Ends with regulation of a downstream cellular process, e.g. transcription. References: PMID:25392484, PMID:27764665 Sources: GOC:bhm Also known as: 5-HT-gated cation-selective signaling pathway, 5-HT-gated cation-selective signalling pathway, 5-hydroxytryptamine-gated cation-selective signaling pathway, 5-hydroxytryptamine-gated cation-selective signalling pathway, serotonin-gated cation-selective signalling pathway Relationships: is_a serotonin receptor signaling pathway [GO:0007210]; is_a ligand-gated ion channel signaling pathway [GO:1990806]; BFO_0000051 GO:0022850